{
  "gene_name": "Exosome complex component RRP45",
  "term_label": "rRNA catabolic process",
  "gene": "UniProtKB:Q06265",
  "term_id": "GO:0016075",
  "gene_symbol": "EXOSC9"
}